{
  "gene_name": "ADP-ribosylation factor-like protein 4C",
  "gene": "UniProtKB:P56559",
  "gene_symbol": "ARL4C",
  "term_label": "intracellular protein transport",
  "term_id": "GO:0006886"
}